{
  "gene": "UniProtKB:Q6WN34",
  "gene_symbol": "CHRDL2",
  "term_label": "negative regulation of BMP signaling pathway",
  "gene_name": "Chordin-like protein 2",
  "term_id": "GO:0030514"
}